{
  "term_id": "GO:0004875",
  "gene_symbol": "FPR2",
  "gene_name": "N-formyl peptide receptor 2",
  "gene": "UniProtKB:P25090",
  "term_label": "complement receptor activity"
}